{
  "gene_name": "Polycystin-2-like protein 1",
  "gene": "UniProtKB:Q9P0L9",
  "term_label": "membrane",
  "term_id": "GO:0016020",
  "gene_symbol": "PKD2L1"
}